{
  "gene_symbol": "LYG2",
  "term_id": "GO:0003796",
  "term_label": "lysozyme activity",
  "gene": "UniProtKB:Q86SG7",
  "gene_name": "Lysozyme g-like protein 2"
}